{
  "gene_symbol": "CTBP2",
  "gene": "UniProtKB:P56545",
  "gene_name": "C-terminal-binding protein 2",
  "term_label": "transcription corepressor activity",
  "term_id": "GO:0003714"
}